{
  "term_label": "DNA-binding transcription factor activity, RNA polymerase II-specific",
  "gene_symbol": "CREB1",
  "term_id": "GO:0000981",
  "gene": "UniProtKB:P16220",
  "gene_name": "Cyclic AMP-responsive element-binding protein 1"
}